{
  "term_id": "GO:0097109",
  "gene_symbol": "NRXN2",
  "gene": "UniProtKB:Q9P2S2",
  "gene_name": "Neurexin-2",
  "term_label": "neuroligin family protein binding"
}